{
  "gene_name": "Intermediate conductance calcium-activated potassium channel protein 4",
  "term_label": "neuronal cell body",
  "term_id": "GO:0043025",
  "gene": "UniProtKB:O15554",
  "gene_symbol": "KCNN4"
}